cytokinesis by cell plate formation [GO:0000911] (biological process) Definition: The process of dividing the cytoplasm of a parent cell where a structure forms in the cytoplasm and grows until reaching the plasma membrane, thereby completely separating the cytoplasms of adjacent progeny cells. An example of this is found in Arabidopsis thaliana. Subtypes: GO:0010235, meristemoid mother cell division [GO:0010443] Sources: GOC:clt Relationships: is a type of cytokinesis [GO:0000910]